{
  "gene_symbol": "TANC2",
  "gene_name": "Protein TANC2",
  "gene": "UniProtKB:Q9HCD6",
  "term_label": "dendritic spine",
  "term_id": "GO:0043197"
}